response to methylphenidate [GO:0036271] (biological process) Sources: GOC:hp, Wikipedia:Methylphenidate Also known as: response to MPD, response to MPH, response to ritalin Note: Note that this term is in the subset of terms that should not be used for direct manual annotation of gene products. It was created to be used for cross-referencing by other ontologies. Direct annotations to this term may be amended during annotation QC. Definition: Any process that results in a change in state or activity of a cell or an organism (in terms of movement, secretion, enzyme production, gene expression, etc.) as a result of a methylphenidate stimulus. Relationships: is a type of response to chemical [GO:0042221]